symbiont-mediated perturbation of host process [GO:0044003] (BP) Definition: A process in which a symbiont alters or subverts a biological process in its host organism. The host is defined as the larger of the organisms involved in a symbiotic interaction. Subtypes: symbiont-mediated perturbation of host response to abiotic stimulus [GO:0033635], GO:0036522, symbiont-mediated perturbation of host cellular process [GO:0044068], GO:0052031, symbiont-mediated modulation of host virulence [GO:0098676], effector-mediated perturbation of host process by symbiont [GO:0140418] Also known as: modulation by symbiont of host system process, regulation by symbiont of host system process, disruption by symbiont of host cell, modification by symbiont of host biological process, modification by symbiont of host morphology or physiology, pathogenesis Sources: GOC:cc Relationships: is a type of GO:0035821; is a type of biological process involved in interaction with host [GO:0051701]